{
  "gene": "UniProtKB:P35557",
  "gene_symbol": "GCK",
  "term_id": "GO:0006006",
  "term_label": "glucose metabolic process",
  "gene_name": "Hexokinase-4"
}